catechol oxidase (dimerizing) activity [GO:0047731] (MF) Definition: Catalysis of the reaction: 4 catechol + 3 O2 = 2 dibenzo[1,4]dioxin-2,3-dione + 6 H2O. Relationships: is a type of oxidoreductase activity, acting on the CH-OH group of donors, oxygen as acceptor [GO:0016899] Also known as: catechol:oxygen oxidoreductase (dimerizing) Sources: EC:1.1.3.14, MetaCyc:CATECHOL-OXIDASE-DIMERIZING-RXN